heart valve development [GO:0003170] (biological process) Sources: GOC:mtg_heart Definition: The progression of a heart valve over time, from its formation to the mature structure. A heart valve is a structure that restricts the flow of blood to different regions of the heart and forms from an endocardial cushion. Relationships: is a type of anatomical structure development [GO:0048856]; is part of heart development [GO:0007507] Subtypes: atrioventricular valve development [GO:0003171], sinoatrial valve development [GO:0003172], ventriculo bulbo valve development [GO:0003173], GO:0003178, semi-lunar valve development [GO:1905314] Also known as: cardiac valve development